{
  "term_id": "UNKNOWN:0002",
  "gene": "UniProtKB:O95476",
  "gene_name": "CTD nuclear envelope phosphatase 1",
  "term_label": "Unknown biological process",
  "gene_symbol": "CTDNEP1"
}